{
  "term_id": "UNKNOWN:0001",
  "gene": "UniProtKB:Q496A3",
  "term_label": "Unknown molecular function",
  "gene_name": "Spermatogenesis-associated serine-rich protein 1",
  "gene_symbol": "SPATS1"
}